{
  "term_id": "GO:0004672",
  "term_label": "protein kinase activity",
  "gene_name": "Ribosomal protein S6 kinase-related protein",
  "gene": "UniProtKB:Q96LW2",
  "gene_symbol": "RSKR"
}